{
  "term_label": "positive regulation of T cell mediated cytotoxicity",
  "gene_name": "HLA class I histocompatibility antigen, alpha chain E",
  "gene": "UniProtKB:P13747",
  "gene_symbol": "HLA-E",
  "term_id": "GO:0001916"
}